{
  "gene_name": "Golgin subfamily A member 8H",
  "term_id": "UNKNOWN:0001",
  "gene": "UniProtKB:P0CJ92",
  "term_label": "Unknown molecular function",
  "gene_symbol": "GOLGA8H"
}